{
  "gene_symbol": "CDX2",
  "gene": "UniProtKB:Q99626",
  "term_label": "regulation of transcription by RNA polymerase II",
  "term_id": "GO:0006357",
  "gene_name": "Homeobox protein CDX-2"
}